{
  "gene_name": "Isopentenyl-diphosphate delta-isomerase 2",
  "term_label": "cytoplasm",
  "gene": "UniProtKB:Q9BXS1",
  "term_id": "GO:0005737",
  "gene_symbol": "IDI2"
}